alpha6-beta4 integrin-Shc-Grb2 complex [GO:0070333] (cellular component) Relationships: is a type of plasma membrane protein complex [GO:0098797] Definition: A protein complex that consists of an alpha6-beta4 integrin complex bound to the adaptor proteins Shc and Grb2. Also known as: ITGA6-ITGB4-SHC-GRB2 complex References: PMID:7556090